quaternary ammonium group:proton symporter activity [GO:0015652] (molecular function) Definition: Enables the transfer of a solute or solutes from one side of a membrane to the other according to the reaction: quaternary ammonium group(out) + H+(out) = quaternary ammonium group(in) + H+(in). Sources: GOC:ai Relationships: is a type of solute:proton symporter activity [GO:0015295]; is a type of quaternary ammonium group transmembrane transporter activity [GO:0015651] Subtypes: GO:0015653 Also known as: quaternary ammonium group:hydrogen symporter activity